{
  "term_label": "Unknown molecular function",
  "gene_symbol": "FAM53B",
  "term_id": "UNKNOWN:0001",
  "gene": "UniProtKB:Q14153",
  "gene_name": "Protein FAM53B"
}